{
  "term_label": "cytidine to uridine editing",
  "gene_name": "DNA dC-dU-editing enzyme APOBEC-3F",
  "gene": "UniProtKB:Q8IUX4",
  "term_id": "GO:0016554",
  "gene_symbol": "APOBEC3F"
}